tuberculosinol biosynthetic process [GO:0035440] (biological process) Also known as: halima-5,6,dien-15-ol biosynthesis, halima-5,6,dien-15-ol biosynthetic process, tuberculosinol biosynthesis Definition: The chemical reactions and pathways resulting in the formation of tuberculosinol (halima-5,6,dien-15-ol), a secondary metabolite in Mycobacteria. Relationships: is a type of diterpenoid biosynthetic process [GO:0016102] Sources: MetaCyc:PWY-5935